{
  "gene": "UniProtKB:Q9NY35",
  "gene_name": "Claudin domain-containing protein 1",
  "term_label": "Unknown cellular component",
  "term_id": "UNKNOWN:0003",
  "gene_symbol": "CLDND1"
}